{
  "term_id": "GO:0007218",
  "gene_symbol": "UTS2R",
  "gene_name": "Urotensin-2 receptor",
  "term_label": "neuropeptide signaling pathway",
  "gene": "UniProtKB:Q9UKP6"
}